{
  "gene_name": "C-C motif chemokine 3",
  "term_label": "CCR chemokine receptor binding",
  "term_id": "GO:0048020",
  "gene_symbol": "CCL3",
  "gene": "UniProtKB:P10147"
}